{
  "gene": "UniProtKB:Q8N819",
  "term_label": "protein serine/threonine phosphatase activity",
  "gene_name": "Probable protein phosphatase 1N",
  "term_id": "GO:0004722",
  "gene_symbol": "PPM1N"
}